{
  "gene_name": "Intraflagellar transport protein 122 homolog",
  "term_id": "GO:0061512",
  "gene_symbol": "IFT122",
  "gene": "UniProtKB:Q9HBG6",
  "term_label": "protein localization to cilium"
}